{
  "gene": "UniProtKB:Q9NWZ3",
  "gene_name": "Interleukin-1 receptor-associated kinase 4",
  "term_label": "Unknown molecular function",
  "gene_symbol": "IRAK4",
  "term_id": "UNKNOWN:0001"
}